{
  "gene": "UniProtKB:O75368",
  "term_id": "GO:0005829",
  "gene_symbol": "SH3BGRL",
  "term_label": "cytosol",
  "gene_name": "Adapter SH3BGRL"
}